{
  "gene": "UniProtKB:P09234",
  "term_id": "GO:0030627",
  "gene_name": "U1 small nuclear ribonucleoprotein C",
  "gene_symbol": "SNRPC",
  "term_label": "pre-mRNA 5'-splice site binding"
}